{
  "gene": "UniProtKB:Q8WZ60",
  "gene_name": "Kelch-like protein 6",
  "gene_symbol": "KLHL6",
  "term_label": "proteasome-mediated ubiquitin-dependent protein catabolic process",
  "term_id": "GO:0043161"
}